{
  "term_label": "RNA polymerase II cis-regulatory region sequence-specific DNA binding",
  "gene_name": "Nuclear factor NF-kappa-B p105 subunit",
  "gene": "UniProtKB:P19838",
  "gene_symbol": "NFKB1",
  "term_id": "GO:0000978"
}